negative regulation of actin nucleation [GO:0051126] (BP) Also known as: down regulation of actin nucleation, down-regulation of actin nucleation, downregulation of actin nucleation, inhibition of actin nucleation Sources: GOC:ai Subtypes: negative regulation of Arp2/3 complex-mediated actin nucleation [GO:0034316] Relationships: is a type of regulation of actin nucleation [GO:0051125]; is a type of negative regulation of cytoskeleton organization [GO:0051494]; is a type of GO:1902904; negatively regulates actin nucleation [GO:0045010] Definition: Any process that stops, prevents, or reduces the frequency, rate or extent of actin nucleation, the initial step in the formation of an actin filament in which actin monomers combine to form a new filament.